{
  "gene": "UniProtKB:Q8N0Y2",
  "term_id": "GO:0000981",
  "term_label": "DNA-binding transcription factor activity, RNA polymerase II-specific",
  "gene_name": "Zinc finger protein 444",
  "gene_symbol": "ZNF444"
}